MLL1/2 complex [GO:0044665] (cellular component) Definition: A protein complex that can methylate lysine-4 of histone H3, and which contains either of the protein subunits MLL1 or MLL2 in human, or equivalent in other species. Relationships: is a type of histone methyltransferase complex [GO:0035097] Also known as: Trx-containing complex References: PMID:21875999 Sources: GOC:sart Subtypes: MLL1 complex [GO:0071339]